{
  "term_label": "cytoplasm",
  "term_id": "GO:0005737",
  "gene": "UniProtKB:P31371",
  "gene_symbol": "FGF9",
  "gene_name": "Fibroblast growth factor 9"
}